{
  "gene_name": "Inositol 1,4,5-trisphosphate receptor type 1",
  "term_label": "inositol 1,4,5 trisphosphate binding",
  "gene_symbol": "ITPR1",
  "gene": "UniProtKB:Q14643",
  "term_id": "GO:0070679"
}